{
  "term_label": "actin filament organization",
  "gene": "UniProtKB:Q9Y5K6",
  "gene_name": "CD2-associated protein",
  "gene_symbol": "CD2AP",
  "term_id": "GO:0007015"
}